{
  "gene_name": "Katanin p80 WD40 repeat-containing subunit B1",
  "gene_symbol": "KATNB1",
  "term_id": "GO:0008352",
  "term_label": "katanin complex",
  "gene": "UniProtKB:Q9BVA0"
}